{
  "term_id": "GO:0016339",
  "gene_symbol": "CDH9",
  "term_label": "calcium-dependent cell-cell adhesion",
  "gene_name": "Cadherin-9",
  "gene": "UniProtKB:Q9ULB4"
}